{
  "term_id": "UNKNOWN:0001",
  "gene": "UniProtKB:Q96JB8",
  "term_label": "Unknown molecular function",
  "gene_name": "MAGUK p55 subfamily member 4",
  "gene_symbol": "MPP4"
}